{
  "gene": "UniProtKB:P30533",
  "term_label": "lipase binding",
  "term_id": "GO:0035473",
  "gene_symbol": "LRPAP1",
  "gene_name": "Alpha-2-macroglobulin receptor-associated protein"
}